myosin filament assembly [GO:0031034] (biological process) Definition: The aggregation, arrangement and bonding together of a filament composed of myosin molecules. Sources: GOC:mah Also known as: myosin polymerization Relationships: is a type of myosin filament organization [GO:0031033]; is a type of protein-containing complex assembly [GO:0065003] Subtypes: GO:0031036, striated muscle myosin thick filament assembly [GO:0071688]